{
  "term_label": "protein folding",
  "gene": "UniProtKB:Q8WVJ2",
  "gene_name": "NudC domain-containing protein 2",
  "gene_symbol": "NUDCD2",
  "term_id": "GO:0006457"
}